vesicle fusion with Golgi medial cisterna membrane [GO:1990671] (biological process) Definition: The joining of the lipid bilayer membrane around a vesicle to the lipid bilayer membrane around the Golgi medial cisterna. This can involve anterograde or retrograde transport vesicles. Relationships: is a type of vesicle fusion with Golgi apparatus [GO:0048280] References: PMID:16038056, PMID:24119662 Sources: GOC:bhm